{
  "gene": "UniProtKB:P0CJ78",
  "term_label": "DNA-binding transcription factor activity",
  "gene_name": "Zinc finger protein 865",
  "gene_symbol": "ZNF865",
  "term_id": "GO:0003700"
}